potassium channel complex [GO:0034705] (cellular component) Definition: An ion channel complex through which potassium ions pass. Sources: GOC:mah Relationships: is a type of cation channel complex [GO:0034703] Subtypes: voltage-gated potassium channel complex [GO:0008076], GO:0008282, GO:0032983, mitochondrial ATP-gated potassium channel complex [GO:0062157]